natural killer cell progenitor differentiation [GO:0002321] (biological process) References: PMID:16551251, PMID:16551264 Sources: GOC:add Relationships: is a type of lymphoid progenitor cell differentiation [GO:0002320] Definition: The process in which a precursor cell type acquires the specialized features of a natural killer cell progenitor.